{
  "gene_name": "Tetratricopeptide repeat protein 31",
  "term_label": "Unknown molecular function",
  "gene_symbol": "TTC31",
  "term_id": "UNKNOWN:0001",
  "gene": "UniProtKB:Q49AM3"
}